phosphatidylcholine metabolic process [GO:0046470] (biological process) Subtypes: 1,2-diacyl-sn-glycero-3-phosphocholine metabolic process [GO:0006653], GO:0006656, GO:0034638, GO:0036151, phosphatidylethanolamine acyl-chain remodeling [GO:0036152] Also known as: phosphatidylcholine metabolism Definition: The chemical reactions and pathways involving phosphatidylcholines, any of a class of glycerophospholipids in which the phosphatidyl group is esterified to the hydroxyl group of choline. They are important constituents of cell membranes. Sources: ISBN:0198506732 Regulation: regulated by regulation of phosphatidylcholine metabolic process [GO:0150172] Relationships: is a type of glycerophospholipid metabolic process [GO:0006650]